{
  "term_label": "deoxyribonucleotide biosynthetic process",
  "term_id": "GO:0009263",
  "gene": "UniProtKB:P23921",
  "gene_symbol": "RRM1",
  "gene_name": "Ribonucleoside-diphosphate reductase large subunit"
}